{
  "gene_symbol": "GPN2",
  "term_id": "UNKNOWN:0002",
  "gene_name": "GPN-loop GTPase 2",
  "term_label": "Unknown biological process",
  "gene": "UniProtKB:Q9H9Y4"
}